hypotonic salinity response [GO:0042539] (biological process) Definition: Any process that results in a change in state or activity of a cell or an organism (in terms of movement, secretion, enzyme production, gene expression, etc.) as a result of detection of, or exposure to, a decrease in the concentration of salt (particularly but not exclusively sodium and chloride ions) in the environment. Sources: GOC:jl Also known as: response to hypotonic salt stress Relationships: is a type of hypotonic response [GO:0006971]; is a type of response to salt stress [GO:0009651] Subtypes: cellular hypotonic salinity response [GO:0071477]